generation of catalytic spliceosome for first transesterification step [GO:0000349] (biological process) Sources: GOC:krc, ISBN:0879695897 Relationships: is_a GO:0022618; is part of spliceosomal conformational changes to generate catalytic conformation [GO:0000393] Definition: Formation of a catalytic spliceosome complex ready to perform the first splicing reaction. This occurs by an ATP-dependent conformational change of the pre-catalytic spliceosome. Also known as: formation of catalytic spliceosome for first transesterification step, U12-type catalytic spliceosome formation for first transesterification step, U2-type catalytic spliceosome formation for first transesterification step, spliceosomal A2-2 complex biosynthesis, spliceosomal A2-2 complex formation, spliceosomal C1 complex biosynthesis, spliceosomal C1 complex formation, catalytic spliceosome assembly for first transesterification step Note: Note that this step represents the formation of the A2-2 complex (yeast) or the C1 complex (mammalian).